{
  "gene": "UniProtKB:O95239",
  "gene_symbol": "KIF4A",
  "term_id": "GO:0051231",
  "gene_name": "Chromosome-associated kinesin KIF4A",
  "term_label": "spindle elongation"
}